protein-glycine ligase activity, elongating [GO:0070737] (molecular function) Definition: Catalysis of the posttranslational transfer of one or more glycine residues to a glycine residue covalently attached to the gamma-carboxyl group of a glutamate residue on a target protein, resulting in the elongation of a polyglycine side chain. Relationships: is a type of GO:0070735 Also known as: protein glycylase activity, elongating References: PMID:19524510 Sources: GOC:mah